mucosa-associated lymphoid tissue development [GO:0048537] (BP) Relationships: is a type of tissue development [GO:0009888]; is a type of hematopoietic or lymphoid organ development [GO:0048534] Subtypes: Peyer's patch development [GO:0048541] Sources: GOC:add, ISBN:0781735149 Also known as: mucosal-associated lymphoid tissue development, BALT development, GALT development, NALT development, bronchial-associated lymphoid tissue development, gut-associated lymphoid tissue development, nasopharyngeal-associated lymphoid tissue development Definition: The process whose specific outcome is the progression of mucosal-associated lymphoid tissue over time, from its formation to the mature structure. Mucosal-associated lymphoid tissue is typically found as nodules associated with mucosal epithelia with distinct internal structures including B- and T-zones for the activation of lymphocytes.